{
  "gene_symbol": "DGKD",
  "term_label": "ATP-dependent diacylglycerol kinase activity",
  "gene_name": "Diacylglycerol kinase delta",
  "term_id": "GO:0004143",
  "gene": "UniProtKB:Q16760"
}